{
  "gene_symbol": "IGKV1D-43",
  "gene": "UniProtKB:A0A0B4J1Z2",
  "gene_name": "Immunoglobulin kappa variable 1D-43",
  "term_label": "immune response",
  "term_id": "GO:0006955"
}